{
  "term_label": "membrane",
  "term_id": "GO:0016020",
  "gene_name": "Polycystin-1-like protein 2",
  "gene_symbol": "PKD1L2",
  "gene": "UniProtKB:Q7Z442"
}